negative regulation of smooth muscle cell differentiation [GO:0051151] (biological process) Subtypes: negative regulation of vascular associated smooth muscle cell differentiation [GO:1905064], negative regulation of ureter smooth muscle cell differentiation [GO:2000062], GO:2000357 Relationships: is a type of negative regulation of muscle cell differentiation [GO:0051148]; is a type of GO:0051150; negatively regulates GO:0051145 Also known as: down regulation of smooth muscle cell differentiation, down-regulation of smooth muscle cell differentiation, downregulation of smooth muscle cell differentiation, inhibition of smooth muscle cell differentiation Definition: Any process that stops, prevents, or reduces the frequency, rate or extent of smooth muscle cell differentiation. Sources: CL:0000192, GOC:ai